vasopressin receptor activity [GO:0005000] (molecular function) Sources: GOC:ai Definition: Combining with vasopressin to initiate a change in cell activity. Relationships: is a type of G protein-coupled peptide receptor activity [GO:0008528] Also known as: vasopressin activated calcium mobilizing receptor activity